{
  "gene_symbol": "DDX55",
  "gene": "UniProtKB:Q8NHQ9",
  "gene_name": "ATP-dependent RNA helicase DDX55",
  "term_label": "Unknown molecular function",
  "term_id": "UNKNOWN:0001"
}